{
  "term_id": "GO:0008017",
  "gene": "UniProtKB:Q9ULI4",
  "term_label": "microtubule binding",
  "gene_symbol": "KIF26A",
  "gene_name": "Kinesin-like protein KIF26A"
}